{
  "gene": "UniProtKB:P00918",
  "gene_name": "Carbonic anhydrase 2",
  "term_label": "apical part of cell",
  "gene_symbol": "CA2",
  "term_id": "GO:0045177"
}